{
  "gene_symbol": "DSPP",
  "term_label": "dentinogenesis",
  "term_id": "GO:0097187",
  "gene_name": "Dentin sialophosphoprotein",
  "gene": "UniProtKB:Q9NZW4"
}